cap-independent translational initiation of linear mRNA [GO:0110017] (biological process) Relationships: is a type of cap-independent translational initiation [GO:0002190] Subtypes: IRES-dependent translational initiation of linear mRNA [GO:0002192] Definition: The process where translation initiation recruits the 40S ribosomal subunits in a cap and 5' end independent fashion before an AUG codon is encountered in an appropriate sequence context to initiate linear mRNA translation. Sources: GOC:kmv